{
  "term_label": "Unknown biological process",
  "gene_name": "RNA-binding protein 27",
  "gene": "UniProtKB:Q9P2N5",
  "gene_symbol": "RBM27",
  "term_id": "UNKNOWN:0002"
}